{
  "term_label": "endoplasmic reticulum membrane",
  "gene_symbol": "HACD2",
  "gene": "UniProtKB:Q6Y1H2",
  "term_id": "GO:0005789",
  "gene_name": "Very-long-chain (3R)-3-hydroxyacyl-CoA dehydratase 2"
}